{
  "gene_symbol": "MROH1",
  "gene": "UniProtKB:Q8NDA8",
  "gene_name": "Maestro heat-like repeat-containing protein family member 1",
  "term_label": "Unknown biological process",
  "term_id": "UNKNOWN:0002"
}